regulation of pole plasm oskar mRNA localization [GO:0007317] (BP) Subtypes: negative regulation of pole plasm oskar mRNA localization [GO:0045855], positive regulation of pole plasm oskar mRNA localization [GO:0045856] Sources: GOC:hb Relationships: is a type of GO:1904580; regulates pole plasm oskar mRNA localization [GO:0045451] Definition: Any process that modulates the frequency, rate or extent of the process in which oskar mRNA is transported to, or maintained in, the oocyte pole plasm. Also known as: regulation of oocyte pole plasm oskar mRNA localization, regulation of pole plasm oskar mRNA localisation